{
  "gene_symbol": "SRARP",
  "term_label": "nuclear estrogen receptor binding",
  "gene": "UniProtKB:Q8NEQ6",
  "gene_name": "Steroid receptor-associated and regulated protein",
  "term_id": "GO:0030331"
}